central nervous system control of baroreceptor feedback [GO:0003019] (biological process) Definition: The neurological process in which nerve impulses arising in the aorta or the carotid sinuses travel to the medulla and reach the nucleus of tractus solaris. Relationships: is a type of nervous system process involved in regulation of systemic arterial blood pressure [GO:0001976]; is part of regulation of systemic arterial blood pressure by carotid sinus baroreceptor feedback [GO:0001978] Sources: GOC:mtg_cardio, ISBN:0323031951